{
  "gene_name": "Acyl-coenzyme A thioesterase 1",
  "term_id": "GO:0006631",
  "term_label": "fatty acid metabolic process",
  "gene": "UniProtKB:Q86TX2",
  "gene_symbol": "ACOT1"
}